{
  "gene_symbol": "HMG20A",
  "term_label": "nucleus",
  "gene": "UniProtKB:Q9NP66",
  "term_id": "GO:0005634",
  "gene_name": "High mobility group protein 20A"
}